{
  "gene_name": "Importin-5",
  "gene": "UniProtKB:O00410",
  "gene_symbol": "IPO5",
  "term_label": "protein import into nucleus",
  "term_id": "GO:0006606"
}